{
  "term_label": "sodium ion homeostasis",
  "gene": "UniProtKB:P55011",
  "term_id": "GO:0055078",
  "gene_name": "Solute carrier family 12 member 2",
  "gene_symbol": "SLC12A2"
}